{
  "gene_name": "Arf-GAP with Rho-GAP domain, ANK repeat and PH domain-containing protein 2",
  "term_id": "GO:0032956",
  "gene": "UniProtKB:Q8WZ64",
  "gene_symbol": "ARAP2",
  "term_label": "regulation of actin cytoskeleton organization"
}